{
  "gene_symbol": "CACNA1A",
  "term_label": "calcium ion import across plasma membrane",
  "term_id": "GO:0098703",
  "gene_name": "Voltage-dependent P_Q-type calcium channel subunit alpha-1A",
  "gene": "UniProtKB:O00555"
}